{
  "gene_name": "Matrix metalloproteinase-28",
  "term_label": "collagen catabolic process",
  "gene": "UniProtKB:Q9H239",
  "gene_symbol": "MMP28",
  "term_id": "GO:0030574"
}